regulation of cellular defense response [GO:0010185] (BP) Definition: Any process that modulates the frequency, rate or extent of cellular defense response. Sources: GOC:sm Subtypes: positive regulation of cellular defense response [GO:0010186], GO:0051245 Relationships: is a type of regulation of defense response [GO:0031347]; regulates cellular defense response [GO:0006968] Also known as: regulation of cellular defence response